{
  "term_label": "RNA binding",
  "term_id": "GO:0003723",
  "gene_symbol": "RPL11",
  "gene_name": "Large ribosomal subunit protein uL5",
  "gene": "UniProtKB:P62913"
}